glycerophosphodiester phosphodiesterase activity [GO:0008889] (molecular function) Relationships: is a type of phosphoric diester hydrolase activity [GO:0008081] Sources: EC:3.1.4.46 Also known as: IgD-binding protein D, gene hpd protein, glycerophosphodiester glycerophosphohydrolase activity, glycerophosphoryl diester phosphodiesterase activity Definition: Catalysis of the reaction: a glycerophosphodiester + H2O = an alcohol + sn-glycerol 3-phosphate.